{
  "gene_symbol": "ITGAL",
  "term_label": "cell-cell adhesion",
  "gene": "UniProtKB:P20701",
  "gene_name": "Integrin alpha-L",
  "term_id": "GO:0098609"
}